trigeminothalamic tract morphogenesis [GO:0021974] (biological process) Sources: GOC:cls, GOC:dgh, GOC:dph, GOC:jid, GO_REF:0000021 Relationships: is_a GO:0021952 Definition: Generation of a long process of a CNS neuron, that carries efferent (outgoing) action potentials from the cell body in spinal cord towards target cells in the thalamus. This axonal process is a member of those that make up the trigeminothalamic tract, one of the major routes of nociceptive and temperature signaling from the face.